positive regulation of iodide transport [GO:1904203] (biological process) Also known as: up regulation of iodide transport, up-regulation of iodide transport, upregulation of iodide transport, activation of iodide transport Relationships: is a type of positive regulation of monoatomic anion transport [GO:1903793]; is a type of regulation of iodide transport [GO:1904201]; positively regulates iodide transport [GO:0015705] Definition: Any process that activates or increases the frequency, rate or extent of iodide transport. References: PMID:20392814 Sources: GOC:TermGenie, GO_REF:0000058 Subtypes: GO:1904214